ciliary necklace [GO:0097538] (cellular component) Definition: A protein complex located on the cilium membrane in the ciliary transition zone; it is connected to the cilium axoneme via Y-shaped links. Relationships: is a type of plasma membrane protein complex [GO:0098797]; is part of GO:0035869; is part of GO:0060170 Also known as: cilial necklace, cilium necklace References: PMID:22653444, PMID:4554367 Sources: GOC:cilia